{
  "gene_symbol": "KCNE2",
  "gene": "UniProtKB:Q9Y6J6",
  "term_id": "GO:0015459",
  "gene_name": "Potassium voltage-gated channel subfamily E member 2",
  "term_label": "potassium channel regulator activity"
}